{
  "term_id": "GO:0061630",
  "gene_symbol": "TRIM49C",
  "gene_name": "Tripartite motif-containing protein 49C",
  "gene": "UniProtKB:P0CI26",
  "term_label": "ubiquitin protein ligase activity"
}